{
  "gene_symbol": "MLF1",
  "term_label": "Unknown molecular function",
  "gene": "UniProtKB:P58340",
  "gene_name": "Myeloid leukemia factor 1",
  "term_id": "UNKNOWN:0001"
}